{
  "gene_name": "Low-density lipoprotein receptor class A domain-containing protein 1",
  "gene": "UniProtKB:Q5T700",
  "gene_symbol": "LDLRAD1",
  "term_label": "Unknown molecular function",
  "term_id": "UNKNOWN:0001"
}